extrahaustorial membrane [GO:0085037] (cellular component) Sources: GOC:pamgo_curators Note: See also: haustorium ; GO:0085035 and extrahaustorial matrix ; GO:0085036. Relationships: is a type of GO:0033644; is part of GO:0020002 Definition: The membrane surrounding the symbiont haustorium during symbiosis, derived from the host plasma membrane.